regulation of skeletal muscle cell proliferation [GO:0014857] (biological process) Sources: CL:0000188, GOC:ef, GOC:mtg_muscle Subtypes: GO:0014842, positive regulation of skeletal muscle cell proliferation [GO:0014858], negative regulation of skeletal muscle cell proliferation [GO:0014859] Relationships: is a type of regulation of cell population proliferation [GO:0042127]; regulates skeletal muscle cell proliferation [GO:0014856] Definition: Any process that modulates the frequency, rate or extent of skeletal muscle cell proliferation.